{
  "term_label": "nuclear pore outer ring",
  "gene": "UniProtKB:Q8NFH4",
  "gene_name": "Nucleoporin Nup37",
  "gene_symbol": "NUP37",
  "term_id": "GO:0031080"
}